{
  "gene_name": "E3 ubiquitin-protein ligase ZFP91",
  "term_id": "GO:0005634",
  "term_label": "nucleus",
  "gene": "UniProtKB:Q96JP5",
  "gene_symbol": "ZFP91"
}